mycofactocin biosynthetic process [GO:0140604] (biological process) References: PMID:21223593, PMID:27312813, PMID:30183269, PMID:30778644, PMID:31381312, PMID:33014324 Relationships: is a type of biosynthetic process [GO:0009058] Definition: The chemical reactions and pathways resulting in the formation of the coenzyme mycofactocin, a variably glycosylated small molecule electron pair carrier derived from the C-terminal valine-tyrosine dipeptide of the ribosomally translated precursor peptide MftA.